{
  "gene_symbol": "SKIL",
  "gene": "UniProtKB:P12757",
  "gene_name": "Ski-like protein",
  "term_id": "GO:0030512",
  "term_label": "negative regulation of transforming growth factor beta receptor signaling pathway"
}